{
  "gene": "UniProtKB:O75051",
  "gene_symbol": "PLXNA2",
  "gene_name": "Plexin-A2",
  "term_id": "GO:0005886",
  "term_label": "plasma membrane"
}